{
  "gene_name": "Probable palmitoyltransferase ZDHHC24",
  "gene": "UniProtKB:Q6UX98",
  "gene_symbol": "ZDHHC24",
  "term_id": "GO:0019706",
  "term_label": "protein-cysteine S-palmitoyltransferase activity"
}